{
  "gene": "UniProtKB:Q9UJX6",
  "gene_symbol": "ANAPC2",
  "term_label": "Unknown molecular function",
  "gene_name": "Anaphase-promoting complex subunit 2",
  "term_id": "UNKNOWN:0001"
}